positive regulation of molecular function [GO:0044093] (biological process) Definition: Any process that activates or increases the rate or extent of a molecular function, an elemental biological activity occurring at the molecular level, such as catalysis or binding. Sources: GO:jl Relationships: is a type of regulation of molecular function [GO:0065009]; positively regulates molecular_function [GO:0003674] Subtypes: positive regulation of transporter activity [GO:0032411], GO:0032781, GO:0043085, positive regulation of DNA-binding transcription factor activity [GO:0051091], positive regulation of binding [GO:0051099]